{
  "gene_name": "Serine_arginine repetitive matrix protein 4",
  "term_id": "GO:0043484",
  "gene": "UniProtKB:A7MD48",
  "gene_symbol": "SRRM4",
  "term_label": "regulation of RNA splicing"
}